{
  "term_label": "nucleus",
  "gene_symbol": "DDX19B",
  "gene_name": "ATP-dependent RNA helicase DDX19B",
  "term_id": "GO:0005634",
  "gene": "UniProtKB:Q9UMR2"
}